{
  "gene_name": "WD repeat domain phosphoinositide-interacting protein 2",
  "gene": "UniProtKB:Q9Y4P8",
  "term_id": "GO:0044804",
  "term_label": "nucleophagy",
  "gene_symbol": "WIPI2"
}